{
  "gene": "UniProtKB:O60635",
  "term_label": "Unknown biological process",
  "gene_symbol": "TSPAN1",
  "term_id": "UNKNOWN:0002",
  "gene_name": "Tetraspanin-1"
}